intracellular polyamine homeostasis [GO:0010509] (biological process) References: PMID:11161802, PMID:9761731 Sources: GOC:dph, GOC:rph, GOC:tb Definition: A homeostatic process involved in the maintenance of a steady state level of polyamine within a cell. Also known as: polyamine homeostasis Relationships: is a type of intracellular chemical homeostasis [GO:0055082]